myosin I light chain binding [GO:0032030] (molecular function) Relationships: is a type of GO:0017024; is a type of myosin light chain binding [GO:0032027] Sources: GOC:mah Definition: Binding to a light chain of a myosin I complex.